response to salicylic acid [GO:0009751] (biological process) Also known as: response to salicylate, response to salicylic acid stimulus Subtypes: detection of salicylic acid stimulus [GO:0009752], cellular response to salicylic acid stimulus [GO:0071446] Relationships: is a type of response to oxygen-containing compound [GO:1901700] Definition: Any process that results in a change in state or activity of a cell or an organism (in terms of movement, secretion, enzyme production, gene expression, etc.) as a result of a salicylic acid stimulus. Sources: GOC:jl